{
  "gene_name": "Transmembrane protein 31",
  "term_label": "Unknown molecular function",
  "term_id": "UNKNOWN:0001",
  "gene_symbol": "TMEM31",
  "gene": "UniProtKB:Q5JXX7"
}